{
  "term_id": "GO:0000978",
  "gene": "UniProtKB:Q96SC8",
  "gene_symbol": "DMRTA2",
  "term_label": "RNA polymerase II cis-regulatory region sequence-specific DNA binding",
  "gene_name": "Doublesex- and mab-3-related transcription factor A2"
}